{
  "gene_symbol": "CD22",
  "term_label": "sialic acid binding",
  "gene_name": "B-cell receptor CD22",
  "term_id": "GO:0033691",
  "gene": "UniProtKB:P20273"
}